aerotaxis [GO:0009454] (biological process) Definition: The directed movement of a motile cell or organism in response to environmental oxygen. Subtypes: negative aerotaxis [GO:0052130], positive aerotaxis [GO:0052131] Also known as: taxis in response to atmospheric oxygen Sources: GOC:jl, ISBN:0192801023 Relationships: is a type of chemotaxis [GO:0006935]; is a type of GO:0009453